{
  "gene": "UniProtKB:A8MW95",
  "term_label": "phosphatidylinositol 3-kinase binding",
  "term_id": "GO:0043548",
  "gene_symbol": "BECN2",
  "gene_name": "Beclin-2"
}